{
  "gene": "UniProtKB:Q495Y7",
  "term_id": "UNKNOWN:0003",
  "gene_symbol": "SPDYE7P",
  "gene_name": "Putative speedy protein E7",
  "term_label": "Unknown cellular component"
}